{
  "term_label": "type I interferon-mediated signaling pathway",
  "term_id": "GO:0060337",
  "gene_symbol": "IFNA8",
  "gene_name": "Interferon alpha-8",
  "gene": "UniProtKB:P32881"
}